{
  "term_label": "regulation of cell migration",
  "term_id": "GO:0030334",
  "gene_symbol": "FGF20",
  "gene_name": "Fibroblast growth factor 20",
  "gene": "UniProtKB:Q9NP95"
}